rhabdomere [GO:0016028] (cellular component) Definition: The specialized microvilli-containing organelle on the apical surfaces of a photoreceptor cell containing the visual pigment rhodopsin and most of the proteins involved in phototransduction. References: PMID:8646774 Sources: GOC:hb, GOC:sart Relationships: is a type of GO:0120025